positive regulation of cellular component biogenesis [GO:0044089] (biological process) Sources: GOC:jl Definition: Any process that activates or increases the frequency, rate or extent of cellular component biogenesis, a process that results in the biosynthesis of constituent macromolecules, assembly, and arrangement of constituent parts of a cellular component. Relationships: is a type of regulation of cellular component biogenesis [GO:0044087]; is a type of positive regulation of cellular process [GO:0048522]; positively regulates cellular component biogenesis [GO:0044085] Subtypes: GO:0031334, GO:0031453, positive regulation of actin filament bundle assembly [GO:0032233], positive regulation of ribosome biogenesis [GO:0090070], positive regulation of inclusion body assembly [GO:0090261], GO:0120034, positive regulation of hyaluranon cable assembly [GO:1900106], positive regulation of extracellular matrix assembly [GO:1901203], GO:1901348, positive regulation of cell junction assembly [GO:1901890], positive regulation of cell septum assembly [GO:1901893], GO:1902117, positive regulation of ascospore-type prospore membrane formation [GO:1903024], positive regulation of exosomal secretion [GO:1903543], positive regulation of t-circle formation [GO:1904431], positive regulation of synaptonemal complex assembly [GO:1905088], GO:1905758, positive regulation of dense core granule biogenesis [GO:2000707], positive regulation of plant-type cell wall cellulose biosynthetic process [GO:2001011]